{
  "term_label": "Unknown biological process",
  "term_id": "UNKNOWN:0002",
  "gene_symbol": "CCDC74A",
  "gene": "UniProtKB:Q96AQ1",
  "gene_name": "Coiled-coil domain-containing protein 74A"
}